response to stimulus [GO:0050896] (biological process) Definition: Any process that results in a change in state or activity of a cell or an organism (in terms of movement, secretion, enzyme production, gene expression, etc.) as a result of a stimulus. The process begins with detection of the stimulus and ends with a change in state or activity or the cell or organism. Regulation: regulated by regulation of response to stimulus [GO:0048583]; RO_0002213 by positive regulation of response to stimulus [GO:0048584]; negatively regulated by negative regulation of response to stimulus [GO:0048585] Relationships: is a type of biological_process [GO:0008150] Note: Note that this term is in the subset of terms that should not be used for direct gene product annotation. Instead, select a child term or, if no appropriate child term exists, please request a new term. Direct annotations to this term may be amended during annotation QC. Also known as: physiological response to stimulus Sources: GOC:ai, GOC:bf Subtypes: response to stress [GO:0006950], immune response [GO:0006955], response to external stimulus [GO:0009605], GO:0009607, response to abiotic stimulus [GO:0009628], response to endogenous stimulus [GO:0009719], response to activity [GO:0014823], response to inactivity [GO:0014854], response to stimulus involved in regulation of muscle adaptation [GO:0014874], response to nutrient levels [GO:0031667], response to chemical [GO:0042221], muscle adaptation [GO:0043500], detection of stimulus [GO:0051606], cellular response to stimulus [GO:0051716], response to redox state [GO:0051775]